{
  "gene_name": "Protein KIBRA",
  "term_id": "GO:0006355",
  "gene": "UniProtKB:Q8IX03",
  "gene_symbol": "WWC1",
  "term_label": "regulation of DNA-templated transcription"
}